postsynaptic recycling endosome membrane [GO:0098944] (cellular component) Definition: The lipid bilayer surrounding a postsynaptic recycling endosome. Sources: GOC:pz Relationships: is a type of postsynaptic endosome membrane [GO:0098895]; is part of postsynaptic recycling endosome [GO:0098837]